{
  "gene_symbol": "ST3GAL3",
  "term_id": "UNKNOWN:0003",
  "gene": "UniProtKB:Q11203",
  "term_label": "Unknown cellular component",
  "gene_name": "CMP-N-acetylneuraminate-beta-1,4-galactoside alpha-2,3-sialyltransferase"
}